{
  "gene_symbol": "UQCR10",
  "term_label": "respiratory chain complex III",
  "gene_name": "Cytochrome b-c1 complex subunit 9",
  "gene": "UniProtKB:Q9UDW1",
  "term_id": "GO:0045275"
}